{
  "gene_symbol": "PNMA6F",
  "term_label": "Unknown cellular component",
  "gene": "UniProtKB:A0A0J9YX94",
  "gene_name": "Paraneoplastic antigen Ma6F",
  "term_id": "UNKNOWN:0003"
}